negative regulation of IP-10 production [GO:0071659] (biological process) Also known as: negative regulation of CXCL10 production, negative regulation of chemokine (C-C motif) ligand 10 production Definition: Any process that stops, prevents, or reduces the frequency, rate, or extent of production of IP-10. Relationships: is a type of negative regulation of chemokine production [GO:0032682]; is a type of regulation of IP-10 production [GO:0071658]; negatively regulates IP-10 production [GO:0071612] Sources: GOC:mah